{
  "term_label": "Hsp90 protein binding",
  "gene": "UniProtKB:O14830",
  "gene_name": "Serine_threonine-protein phosphatase with EF-hands 2",
  "gene_symbol": "PPEF2",
  "term_id": "GO:0051879"
}